{
  "term_label": "antigen processing and presentation, endogenous lipid antigen via MHC class Ib",
  "gene_name": "T-cell surface glycoprotein CD1c",
  "gene_symbol": "CD1C",
  "gene": "UniProtKB:P29017",
  "term_id": "GO:0048006"
}